{
  "term_id": "GO:0016180",
  "gene": "UniProtKB:Q5TA45",
  "gene_symbol": "INTS11",
  "gene_name": "Integrator complex subunit 11",
  "term_label": "snRNA processing"
}